proton binding [GO:1901691] (molecular function) Sources: GOC:TermGenie Also known as: hydrogen ion binding Definition: Binding to proton. Relationships: is a type of cation binding [GO:0043169]